{
  "gene_name": "LIM homeobox transcription factor 1-beta",
  "term_id": "GO:0006357",
  "term_label": "regulation of transcription by RNA polymerase II",
  "gene": "UniProtKB:O60663",
  "gene_symbol": "LMX1B"
}